{
  "gene_name": "Centriolar satellite-associated tubulin polyglutamylase complex regulator 1",
  "gene": "UniProtKB:Q9H6J7",
  "term_id": "UNKNOWN:0001",
  "term_label": "Unknown molecular function",
  "gene_symbol": "CSTPP1"
}